{
  "gene": "UniProtKB:A8MXV6",
  "gene_symbol": "CDRT15L2",
  "term_id": "UNKNOWN:0002",
  "term_label": "Unknown biological process",
  "gene_name": "CMT1A duplicated region transcript 15 protein-like protein"
}